{
  "gene": "UniProtKB:Q8TCQ1",
  "term_label": "late endosome membrane",
  "gene_name": "E3 ubiquitin-protein ligase MARCHF1",
  "gene_symbol": "MARCHF1",
  "term_id": "GO:0031902"
}